electron transport chain [GO:0022900] (biological process) Subtypes: photosynthetic electron transport chain [GO:0009767], GO:0022904, P450-containing electron transport chain [GO:0140647] Sources: GOC:mtg_electron_transport Relationships: is_a generation of precursor metabolites and energy [GO:0006091] Definition: A process in which a series of electron carriers operate together to transfer electrons from donors to any of several different terminal electron acceptors.